{
  "gene_symbol": "GLB1",
  "gene_name": "Beta-galactosidase",
  "term_label": "beta-galactosidase activity",
  "term_id": "GO:0004565",
  "gene": "UniProtKB:P16278"
}